{
  "term_label": "Unknown biological process",
  "gene_name": "Cilia- and flagella-associated protein 45",
  "gene_symbol": "CFAP45",
  "gene": "UniProtKB:Q9UL16",
  "term_id": "UNKNOWN:0002"
}